{
  "term_id": "GO:0051017",
  "gene_symbol": "PLS3",
  "gene_name": "Plastin-3",
  "gene": "UniProtKB:P13797",
  "term_label": "actin filament bundle assembly"
}